sodium:proton antiporter activity involved in regulation of cardiac muscle cell membrane potential [GO:0086040] (molecular function) Sources: GOC:BHF, GOC:mtg_cardiac_conduct_nov11 Also known as: sodium:hydrogen antiporter activity involved in regulation of cardiac muscle cell membrane potential Relationships: is a type of sodium:proton antiporter activity [GO:0015385]; is part of regulation of cardiac muscle cell membrane potential [GO:0086036] Definition: Enables the transfer of a solute or solutes from one side of a cardiac muscle cell membrane to the other according to the reaction: Na+(out) + H+(in) = Na+(in) + H+(out). This transfer contributes to the regulation of the cardiac muscle cell plasma membrane potential.